{
  "term_id": "GO:0000981",
  "term_label": "DNA-binding transcription factor activity, RNA polymerase II-specific",
  "gene": "UniProtKB:Q86Y25",
  "gene_name": "Zinc finger protein 354C",
  "gene_symbol": "ZNF354C"
}